regulation of epithelial cell proliferation involved in mammary gland bud elongation [GO:0060651] (biological process) References: PMID:12558599 Sources: GOC:dph Definition: Any process that modulates the frequency, rate or extent of mammary gland bud epithelial cell proliferation that results in the elongation of the bud. Relationships: is a type of regulation of mammary gland epithelial cell proliferation [GO:0033599]; is a type of GO:2000027; regulates epithelial cell proliferation involved in mammary gland bud elongation [GO:0060650]